{
  "gene_symbol": "PTCRA",
  "term_id": "UNKNOWN:0001",
  "gene_name": "Pre T-cell antigen receptor alpha",
  "term_label": "Unknown molecular function",
  "gene": "UniProtKB:Q6ISU1"
}